{
  "term_label": "defense response to protozoan",
  "gene_name": "Guanylate-binding protein 2",
  "term_id": "GO:0042832",
  "gene_symbol": "GBP2",
  "gene": "UniProtKB:P32456"
}